{
  "gene_symbol": "ZNF337",
  "gene": "UniProtKB:Q9Y3M9",
  "term_label": "regulation of transcription by RNA polymerase II",
  "term_id": "GO:0006357",
  "gene_name": "Zinc finger protein 337"
}